{
  "term_id": "GO:0043197",
  "gene": "UniProtKB:P0DJJ0",
  "term_label": "dendritic spine",
  "gene_name": "SLIT-ROBO Rho GTPase-activating protein 2C",
  "gene_symbol": "SRGAP2C"
}